bilobe structure [GO:0120120] (CC) Also known as: kinetoplastid flagellar hook complex References: PMID:22327007, PMID:22445359, PMID:26540076 Note: Note that we deem cilium and microtubule-based flagellum to be equivalent; the primary term name reflects frequency of use. Relationships: is a type of cellular anatomical structure [GO:0110165]; is part of GO:0005856 Definition: A cytoskeletal structure in some kinetoplastid species linking the structures of the ciliary pocket collar and the flagellum attachment zone (aka cilium attachment zone).